{
  "term_id": "GO:0019226",
  "gene_name": "Voltage-dependent calcium channel gamma-2 subunit",
  "term_label": "transmission of nerve impulse",
  "gene_symbol": "CACNG2",
  "gene": "UniProtKB:Q9Y698"
}